RNA polymerase II promoter clearance [GO:0001111] (biological process) Definition: A process that mediates the transition from the initiation to the elongation phases of transcription by RNA polymerase II, generally including a conformational change from the initiation conformation to the elongation conformation. Promoter clearance often involves breaking contact with transcription factors involved only in the initiation phase and making contacts with elongation specific factors. References: PMID:15020047, PMID:22982364, PMID:31628251 Sources: GOC:txnOH Regulation: regulated by GO:0140845; positively regulated by GO:0140846; negatively regulated by negative regulation of promoter clearance from RNA polymerase II promoter [GO:0140847] Also known as: promoter clearance from RNA polymerase II promoter, promoter escape from RNA polymerase II promoter, promoter-paused RNA polymerase II release Relationships: is a type of promoter clearance during DNA-templated transcription [GO:0001109]; is part of transcription by RNA polymerase II [GO:0006366]